{
  "term_label": "cellular response to amino acid starvation",
  "term_id": "GO:0034198",
  "gene_name": "E3 ubiquitin-protein ligase RNF152",
  "gene": "UniProtKB:Q8N8N0",
  "gene_symbol": "RNF152"
}